{
  "term_label": "Unknown molecular function",
  "gene_name": "Immunoglobulin lambda variable 3-10",
  "gene_symbol": "IGLV3-10",
  "gene": "UniProtKB:A0A075B6K4",
  "term_id": "UNKNOWN:0001"
}